viral release via disruption of host outer membrane [GO:0090680] (biological process) Also known as: disruption by virus of host outer membrane Relationships: is a type of viral release from host cell by cytolysis [GO:0044659]; has part GO:0051673 References: PMID:17900620 Definition: The dissemination of mature viral particles from a host cell via the destabilization of the cell outer membrane.